L-arginine transmembrane import into vacuole [GO:0090518] (biological process) Definition: The directed movement of L-arginine into the vacuole across the vacuolar membrane. Relationships: is a type of GO:0034490; is a type of L-arginine transmembrane transport [GO:1903826] Also known as: arginine transmembrane import into vacuole, vacuolar arginine import Sources: GOC:al